negative regulation of receptor-mediated virion attachment to host cell [GO:1902735] (biological process) References: PMID:18385238 Sources: GOC:TermGenie, GOC:als, GO_REF:0000058 Relationships: is a type of negative regulation of biological process [GO:0048519]; is_a regulation of receptor-mediated virion attachment to host cell [GO:1902734]; negatively regulates receptor-mediated virion attachment to host cell [GO:0046813] Definition: Any process that stops, prevents or reduces the frequency, rate or extent of receptor-mediated virion attachment to host cell. Also known as: down regulation of receptor-mediated virion attachment to host cell, down regulation of virion attachment, binding of host cell surface receptor, down-regulation of receptor-mediated virion attachment to host cell, down-regulation of virion attachment, binding of host cell surface receptor, downregulation of receptor-mediated virion attachment to host cell, downregulation of virion attachment, binding of host cell surface receptor, negative regulation of virion attachment, binding of host cell surface receptor, inhibition of receptor-mediated virion attachment to host cell, inhibition of virion attachment, binding of host cell surface receptor